{
  "gene_name": "Inactive ubiquitin thioesterase OTULINL",
  "gene_symbol": "OTULINL",
  "term_id": "GO:0005737",
  "gene": "UniProtKB:Q9NUU6",
  "term_label": "cytoplasm"
}